{
  "gene": "UniProtKB:P30837",
  "term_label": "mitochondrion",
  "term_id": "GO:0005739",
  "gene_symbol": "ALDH1B1",
  "gene_name": "Aldehyde dehydrogenase X, mitochondrial"
}